{
  "gene": "UniProtKB:O60271",
  "term_label": "MAP-kinase scaffold activity",
  "term_id": "GO:0005078",
  "gene_symbol": "SPAG9",
  "gene_name": "C-Jun-amino-terminal kinase-interacting protein 4"
}